{
  "term_id": "GO:0000902",
  "gene_symbol": "CYFIP2",
  "gene": "UniProtKB:Q96F07",
  "term_label": "cell morphogenesis",
  "gene_name": "Cytoplasmic FMR1-interacting protein 2"
}